dUDP metabolic process [GO:0046077] (biological process) Also known as: dUDP metabolism Sources: GOC:go_curators Subtypes: dUDP biosynthetic process [GO:0006227], dUDP catabolic process [GO:0006257] Definition: The chemical reactions and pathways involving dUDP, deoxyuridine (5'-)diphosphate. Relationships: is a type of pyrimidine deoxyribonucleoside diphosphate metabolic process [GO:0009196]; is a type of GO:0009219